{
  "gene_symbol": "TP53I13",
  "term_label": "Unknown biological process",
  "term_id": "UNKNOWN:0002",
  "gene": "UniProtKB:Q8NBR0",
  "gene_name": "Tumor protein p53-inducible protein 13"
}